tetrapyrrole biosynthetic process [GO:0033014] (biological process) Relationships: is a type of biosynthetic process [GO:0009058]; is a type of tetrapyrrole metabolic process [GO:0033013] Also known as: tetrapyrrole anabolism, tetrapyrrole biosynthesis, tetrapyrrole formation, tetrapyrrole synthesis Regulation: RO_0002211 by regulation of tetrapyrrole biosynthetic process [GO:1901463]; negatively regulated by GO:1901464; positively regulated by positive regulation of tetrapyrrole biosynthetic process [GO:1901465] Subtypes: porphyrin-containing compound biosynthetic process [GO:0006779], GO:0009236, GO:0010024, tetrapyrrole biosynthetic process from glutamate [GO:0033526], tetrapyrrole biosynthetic process from glycine and succinyl-CoA [GO:0033527], GO:0046140, GO:0140609 Definition: The chemical reactions and pathways leading to the formation of tetrapyrroles, natural pigments containing four pyrrole rings joined by one-carbon units linking position 2 of one pyrrole ring to position 5 of the next. Sources: GOC:mah